closure of optic fissure [GO:0061386] (biological process) Also known as: closure or choriod fissure Relationships: is a type of morphogenesis of an epithelial sheet [GO:0002011]; is part of GO:0002072 Definition: The closure of the temporary ventral gap in the optic cup that contributes to its shaping. Sources: GOC:dph